{
  "gene_name": "Retinoic acid receptor RXR-alpha",
  "term_label": "nuclear receptor activity",
  "term_id": "GO:0004879",
  "gene": "UniProtKB:P19793",
  "gene_symbol": "RXRA"
}